{
  "gene_name": "Kinesin-like protein KIF1C",
  "term_id": "GO:0030424",
  "gene": "UniProtKB:O43896",
  "gene_symbol": "KIF1C",
  "term_label": "axon"
}